{
  "term_id": "GO:0005634",
  "term_label": "nucleus",
  "gene": "UniProtKB:A6NF83",
  "gene_symbol": "NUPR2",
  "gene_name": "Nuclear protein 2"
}